cytoplasmic side of transport vesicle membrane [GO:0098539] (cellular component) Sources: GOC:ab Subtypes: cytoplasmic side of trans-Golgi network transport vesicle membrane [GO:0098541] Definition: The side (leaflet) of the transport vesicle membrane that faces the cytoplasm. Also known as: external side of transport vesicle membrane Relationships: is a type of cytoplasmic side of membrane [GO:0098562]; is part of GO:0030658